{
  "gene_symbol": "IGHG2",
  "term_id": "GO:0042571",
  "term_label": "immunoglobulin complex, circulating",
  "gene": "UniProtKB:P01859",
  "gene_name": "Immunoglobulin heavy constant gamma 2"
}